negative regulation of antigen processing and presentation of peptide antigen [GO:0002584] (biological process) Sources: GOC:add Also known as: down regulation of antigen processing and presentation of peptide antigen, down-regulation of antigen processing and presentation of peptide antigen, downregulation of antigen processing and presentation of peptide antigen, negative regulation of peptide antigen processing and presentation, inhibition of antigen processing and presentation of peptide antigen Definition: Any process that stops, prevents, or reduces the frequency, rate, or extent of antigen processing and presentation of peptide antigen. Subtypes: negative regulation of antigen processing and presentation of peptide antigen via MHC class II [GO:0002587], GO:0002590, negative regulation of antigen processing and presentation of peptide antigen via MHC class Ib [GO:0002596], negative regulation of proteolysis associated with antigen processing and presentation [GO:0002629], negative regulation of peptide antigen transport [GO:1901040] Relationships: is_a negative regulation of antigen processing and presentation [GO:0002578]; is_a regulation of antigen processing and presentation of peptide antigen [GO:0002583]; negatively regulates antigen processing and presentation of peptide antigen [GO:0048002]